{
  "gene": "UniProtKB:Q9NZM3",
  "term_id": "GO:0005737",
  "gene_name": "Intersectin-2",
  "term_label": "cytoplasm",
  "gene_symbol": "ITSN2"
}